ribonuclease MRP complex [GO:0000172] (cellular component) Definition: A ribonucleoprotein complex that contains an RNA molecule of the snoRNA family, and cleaves the rRNA precursor as part of rRNA transcript processing. It also has other roles: In S. cerevisiae it is involved in cell cycle-regulated degradation of daughter cell-specific mRNAs, while in mammalian cells it also enters the mitochondria and processes RNAs to create RNA primers for DNA replication. Also known as: RNase MRP complex, ribonuclease mitochondrial RNA processing complex Relationships: is a type of GO:0005732; is a type of endoribonuclease complex [GO:1902555] References: PMID:10690410, PMID:14729943, PMID:7510714 Sources: GOC:sgd_curators